{
  "term_label": "protein targeting to peroxisome",
  "gene": "UniProtKB:Q86WA8",
  "gene_symbol": "LONP2",
  "gene_name": "Lon protease homolog 2, peroxisomal",
  "term_id": "GO:0006625"
}